{
  "term_id": "GO:0005737",
  "gene": "UniProtKB:P32019",
  "gene_symbol": "INPP5B",
  "term_label": "cytoplasm",
  "gene_name": "Type II inositol 1,4,5-trisphosphate 5-phosphatase"
}